{
  "gene": "UniProtKB:Q9Y315",
  "gene_name": "Deoxyribose-phosphate aldolase",
  "term_label": "deoxyribonucleotide catabolic process",
  "term_id": "GO:0009264",
  "gene_symbol": "DERA"
}